{
  "gene_symbol": "VPS45",
  "term_label": "vesicle-mediated transport",
  "gene_name": "Vacuolar protein sorting-associated protein 45",
  "term_id": "GO:0016192",
  "gene": "UniProtKB:Q9NRW7"
}